mesodermal cell fate determination [GO:0007500] (biological process) Relationships: is_a cell fate determination [GO:0001709]; is part of GO:0001710 Sources: GOC:go_curators, ISBN:0878932437 Note: Note that this term was 'mesoderm determination'. Changed string to make more consistent with parent term 'cell fate determination'. Definition: The cell fate determination process in which a cell becomes capable of differentiating autonomously into a mesoderm cell regardless of its environment; upon determination, the cell fate cannot be reversed. Regulation: regulated by GO:0048334; negatively regulated by negative regulation of mesodermal cell fate determination [GO:0048335]; positively regulated by GO:0048336 Subtypes: axial mesodermal cell fate determination [GO:0048323], paraxial mesodermal cell fate determination [GO:0048344], GO:0048373, intermediate mesodermal cell fate determination [GO:0048394] Also known as: mesoderm cell fate determination